{
  "gene": "UniProtKB:A0A494C0Z2",
  "term_id": "UNKNOWN:0002",
  "gene_symbol": "SPDYE13",
  "term_label": "Unknown biological process",
  "gene_name": "Putative speedy protein E13"
}